acetaldehyde dehydrogenase (acetylating) activity [GO:0008774] (molecular function) Sources: EC:1.2.1.10 Also known as: ADA, DmpF, acetaldehyde:NAD+ oxidoreductase (CoA-acetylating), acylating acetaldehyde dehydrogenase activity, aldehyde dehydrogenase (acylating) activity Relationships: is a type of oxidoreductase activity, acting on the aldehyde or oxo group of donors, NAD or NADP as acceptor [GO:0016620] Definition: Catalysis of the reaction: acetaldehyde + CoA + NAD+ = acetyl-CoA + NADH + H+.